{
  "term_label": "cell-cell adhesion mediated by cadherin",
  "gene": "UniProtKB:P55287",
  "gene_name": "Cadherin-11",
  "term_id": "GO:0044331",
  "gene_symbol": "CDH11"
}